{
  "gene": "UniProtKB:Q8TD10",
  "term_label": "Unknown molecular function",
  "gene_symbol": "MIPOL1",
  "term_id": "UNKNOWN:0001",
  "gene_name": "Mirror-image polydactyly gene 1 protein"
}